{
  "gene_symbol": "TAS2R36",
  "term_label": "Unknown biological process",
  "gene_name": "Putative taste receptor type 2 member 36",
  "term_id": "UNKNOWN:0002",
  "gene": "UniProtKB:P0DTE0"
}